negative regulation of retinal ganglion cell axon guidance [GO:0090260] (biological process) Also known as: axon growth cone collapse Note: Note that growth cone collapse has been observed only in assays performed in vitro. Definition: Any process that decreases the frequency, rate, or extent of retinal ganglion cell axon guidance, the process in which the migration of an axon growth cone of a retinal ganglion cell (RGC) is directed to its target in the brain in response to a combination of attractive and repulsive cues. Sources: GOC:tb, GOC:yaf Relationships: is a type of GO:0090259; is a type of negative regulation of axon guidance [GO:1902668]; RO_0002212 retinal ganglion cell axon guidance [GO:0031290]